{
  "term_id": "GO:0043536",
  "gene_symbol": "AKT3",
  "gene_name": "RAC-gamma serine_threonine-protein kinase",
  "gene": "UniProtKB:Q9Y243",
  "term_label": "positive regulation of blood vessel endothelial cell migration"
}